{
  "gene": "UniProtKB:O95996",
  "term_id": "GO:0030877",
  "term_label": "beta-catenin destruction complex",
  "gene_name": "Adenomatous polyposis coli protein 2",
  "gene_symbol": "APC2"
}